response to (R)-carnitine [GO:0061959] (biological process) Definition: Any process that results in a change in state or activity of a cell or an organism (in terms of movement, secretion, enzyme production, gene expression, etc.) as a result of an (R)-carnitine stimulus. References: PMID:28102299 Also known as: response to L-carnitine Relationships: is a type of response to nitrogen compound [GO:1901698]